sodium ion import across plasma membrane [GO:0098719] (biological process) Definition: The directed movement of sodium ions from outside of a cell, across the plasma membrane and into the cytosol. Sources: GOC:dos Also known as: sodium import, sodium ion import into cell, sodium ion import Relationships: is a type of sodium ion transmembrane transport [GO:0035725]; is a type of inorganic cation import across plasma membrane [GO:0098659] Regulation: regulated by regulation of sodium ion import across plasma membrane [GO:1903782]; negatively regulated by GO:1903783; positively regulated by positive regulation of sodium ion import across plasma membrane [GO:1903784]